{
  "term_label": "G protein-coupled receptor binding",
  "gene_name": "Guanine nucleotide-binding protein subunit alpha-11",
  "gene": "UniProtKB:P29992",
  "term_id": "GO:0001664",
  "gene_symbol": "GNA11"
}